{
  "gene_name": "Transcription factor E2F2",
  "term_label": "regulation of transcription by RNA polymerase II",
  "gene": "UniProtKB:Q14209",
  "gene_symbol": "E2F2",
  "term_id": "GO:0006357"
}